{
  "gene": "UniProtKB:P25090",
  "gene_symbol": "FPR2",
  "term_label": "complement receptor mediated signaling pathway",
  "term_id": "GO:0002430",
  "gene_name": "N-formyl peptide receptor 2"
}